{
  "gene": "UniProtKB:P33991",
  "term_label": "nucleus",
  "gene_symbol": "MCM4",
  "term_id": "GO:0005634",
  "gene_name": "DNA replication licensing factor MCM4"
}